{
  "term_id": "GO:0000045",
  "gene": "UniProtKB:Q5BJD5",
  "gene_name": "Transmembrane protein 41B",
  "term_label": "autophagosome assembly",
  "gene_symbol": "TMEM41B"
}